asperthecin biosynthetic process [GO:0036184] (BP) Also known as: asperthecin biosynthesis, asperthecin formation, asperthecin synthesis Relationships: is a type of asperthecin metabolic process [GO:0036182]; is a type of ketone biosynthetic process [GO:0042181]; is a type of secondary metabolite biosynthetic process [GO:0044550]; is_a phenol-containing compound biosynthetic process [GO:0046189] Regulation: RO_0002211 by regulation of asperthecin biosynthetic process [GO:1900379]; negatively regulated by negative regulation of asperthecin biosynthetic process [GO:1900380]; positively regulated by positive regulation of asperthecin biosynthetic process [GO:1900381] Sources: GOC:di Definition: The chemical reactions and pathways resulting in the formation of asperthecin, an anthraquinone pigment obtained from the mould Aspergillus nidulans.